protein autoprocessing [GO:0016540] (biological process) Relationships: is a type of GO:0016485 Definition: Processing which a protein carries out itself. This involves actions such as the autolytic removal of residues to generate the mature form of the protein. References: PMID:9335337 Sources: GOC:ai